negative regulation of cation transmembrane transport [GO:1904063] (biological process) Definition: Any process that stops, prevents or reduces the frequency, rate or extent of cation transmembrane transport. Relationships: is a type of negative regulation of monoatomic ion transmembrane transport [GO:0034766]; is a type of regulation of monoatomic cation transmembrane transport [GO:1904062]; RO_0002212 monoatomic cation transmembrane transport [GO:0098655] Also known as: down regulation of cation transmembrane transport, down-regulation of cation transmembrane transport, downregulation of cation transmembrane transport, inhibition of cation transmembrane transport References: PMID:15304482 Sources: GOC:TermGenie, GO_REF:0000058 Subtypes: negative regulation of iron ion transmembrane transport [GO:0034760], GO:0071583, negative regulation of potassium ion transmembrane transport [GO:1901380], negative regulation of synaptic vesicle lumen acidification [GO:1901547], negative regulation of sodium ion transmembrane transport [GO:1902306], GO:1902312, negative regulation of calcium ion transmembrane transport [GO:1903170]